{
  "term_id": "GO:0003735",
  "gene": "UniProtKB:P62891",
  "term_label": "structural constituent of ribosome",
  "gene_name": "Large ribosomal subunit protein eL39",
  "gene_symbol": "RPL39"
}